{
  "gene_symbol": "CYP4X1",
  "term_id": "UNKNOWN:0003",
  "gene": "UniProtKB:Q8N118",
  "gene_name": "Cytochrome P450 4X1",
  "term_label": "Unknown cellular component"
}